regulation of metal ion transport [GO:0010959] (biological process) Definition: Any process that modulates the frequency, rate, or extent of metal ion transport. Metal ion transport is the directed movement of metal ions, any metal ion with an electric charge, into, out of or within a cell, or between cells, by means of some agent such as a transporter or pore. Sources: GOC:dph, GOC:tb Relationships: is a type of GO:0043269; regulates GO:0030001 Subtypes: regulation of sodium ion transport [GO:0002028], regulation of iron ion transport [GO:0034756], GO:0043266, regulation of calcium ion transport [GO:0051924], regulation of zinc ion transport [GO:0071579], regulation of copper ion transmembrane transport [GO:1902311]